{
  "gene": "UniProtKB:Q9NYV8",
  "gene_name": "Taste receptor type 2 member 14",
  "gene_symbol": "TAS2R14",
  "term_id": "GO:0033038",
  "term_label": "bitter taste receptor activity"
}